{
  "term_id": "GO:0006357",
  "gene_name": "Forkhead box protein D4-like 6",
  "term_label": "regulation of transcription by RNA polymerase II",
  "gene": "UniProtKB:Q3SYB3",
  "gene_symbol": "FOXD4L6"
}